{
  "term_id": "GO:0007010",
  "gene_symbol": "ARHGAP10",
  "gene": "UniProtKB:A1A4S6",
  "gene_name": "Rho GTPase-activating protein 10",
  "term_label": "cytoskeleton organization"
}